{
  "term_id": "UNKNOWN:0002",
  "term_label": "Unknown biological process",
  "gene": "UniProtKB:Q14236",
  "gene_symbol": "DIAPH2-AS1",
  "gene_name": "Early lymphoid activation gene protein"
}